{
  "gene_name": "Dynein regulatory complex subunit 4",
  "term_id": "GO:0045880",
  "gene": "UniProtKB:O95995",
  "term_label": "positive regulation of smoothened signaling pathway",
  "gene_symbol": "GAS8"
}